{
  "term_label": "cytoplasm",
  "gene_symbol": "MROH5",
  "gene": "UniProtKB:Q6ZUA9",
  "gene_name": "Maestro heat-like repeat family member 5",
  "term_id": "GO:0005737"
}